{
  "term_id": "UNKNOWN:0003",
  "gene_symbol": "IGHV1-2",
  "term_label": "Unknown cellular component",
  "gene": "UniProtKB:P23083",
  "gene_name": "Immunoglobulin heavy variable 1-2"
}